{
  "gene_symbol": "SYNE2",
  "term_id": "GO:0031965",
  "term_label": "nuclear membrane",
  "gene_name": "Nesprin-2",
  "gene": "UniProtKB:Q8WXH0"
}